{
  "term_id": "GO:0023052",
  "term_label": "signaling",
  "gene_name": "DCC-interacting protein 13-beta",
  "gene_symbol": "APPL2",
  "gene": "UniProtKB:Q8NEU8"
}